cell chemotaxis involved in Malpighian tubule morphogenesis [GO:0061352] (biological process) Definition: The directed movement of the outgrowing Malpighian tubule guided by specific chemical cues/signals. Movement may be towards a guidance cue (positive chemotaxis) or away from it (negative chemotaxis). Guidance contributes to the final positioning of the tubule. Relationships: is a type of GO:0060326; is_a GO:0061334 Sources: GOC:dph, GOC:mtg_kidney_jan10